immunological synapse [GO:0001772] (cellular component) Definition: An area of close contact between a lymphocyte (T-, B-, or natural killer cell) and a target cell formed through the clustering of particular signaling and adhesion molecules and their associated membrane rafts on both the lymphocyte and the target cell and facilitating activation of the lymphocyte, transfer of membrane from the target cell to the lymphocyte, and in some situations killing of the target cell through release of secretory granules and/or death-pathway ligand-receptor interaction. Relationships: is a type of cellular anatomical structure [GO:0110165]; is part of plasma membrane [GO:0005886] References: PMID:11244041, PMID:11376300 Sources: GOC:mgi_curators Also known as: supramolecular activation cluster, c-SMAC